{
  "gene_symbol": "ZDHHC13",
  "gene_name": "Palmitoyltransferase ZDHHC13",
  "term_id": "UNKNOWN:0001",
  "gene": "UniProtKB:Q8IUH4",
  "term_label": "Unknown molecular function"
}